{
  "term_id": "UNKNOWN:0002",
  "term_label": "Unknown biological process",
  "gene_name": "Uncharacterized protein C17orf50",
  "gene": "UniProtKB:Q8WW18",
  "gene_symbol": "C17orf50"
}